{
  "gene": "UniProtKB:Q02338",
  "term_label": "steroid metabolic process",
  "term_id": "GO:0008202",
  "gene_name": "D-beta-hydroxybutyrate dehydrogenase, mitochondrial",
  "gene_symbol": "BDH1"
}